{
  "gene_name": "Olfactory receptor 5V1",
  "gene_symbol": "OR5V1",
  "gene": "UniProtKB:Q9UGF6",
  "term_label": "detection of chemical stimulus involved in sensory perception of smell",
  "term_id": "GO:0050911"
}